{
  "gene_name": "Epsilon-sarcoglycan",
  "gene": "UniProtKB:O43556",
  "term_id": "GO:0016012",
  "gene_symbol": "SGCE",
  "term_label": "sarcoglycan complex"
}